leaf abscission [GO:0060866] (biological process) Sources: GOC:dph, GOC:sdb_2009, GOC:tb Definition: The controlled shedding of a leaf. Relationships: is a type of GO:0009838